{
  "gene_name": "Cadherin-19",
  "term_id": "GO:0016477",
  "term_label": "cell migration",
  "gene": "UniProtKB:Q9H159",
  "gene_symbol": "CDH19"
}